{
  "gene_name": "Selenocysteine insertion sequence-binding protein 2-like",
  "gene_symbol": "SECISBP2L",
  "term_label": "ribonucleoprotein complex",
  "gene": "UniProtKB:Q93073",
  "term_id": "GO:1990904"
}